regulation of vesicle transport along microtubule [GO:1901608] (biological process) Subtypes: GO:1901609, positive regulation of vesicle transport along microtubule [GO:1901610], regulation of anterograde dense core granule transport [GO:1901951], regulation of retrograde dense core granule transport [GO:1901954], regulation of anterograde synaptic vesicle transport [GO:1903742] Also known as: regulation of microtubule-based vesicle localization Relationships: is a type of regulation of organelle transport along microtubule [GO:1902513]; RO_0002211 vesicle transport along microtubule [GO:0047496] Sources: GOC:TermGenie Definition: Any process that modulates the frequency, rate or extent of vesicle transport along microtubule.